interleukin-17F production [GO:0097088] (BP) Sources: GOC:rv, Wikipedia:Interleukin_17 Definition: The appearance of interleukin-17F due to biosynthesis or secretion following a cellular stimulus, resulting in an increase in its intracellular or extracellular levels. Relationships: is a type of interleukin-17 production [GO:0032620] Also known as: IL-17F production